{
  "gene_name": "Olfactory receptor 5M9",
  "gene_symbol": "OR5M9",
  "term_label": "olfactory receptor activity",
  "term_id": "GO:0004984",
  "gene": "UniProtKB:Q8NGP3"
}